4-amino-3-isothiazolidinone biosynthetic process [GO:0048107] (biological process) Relationships: is a type of sulfur compound biosynthetic process [GO:0044272] Definition: The chemical reactions and pathways resulting in the formation of 4-amino-3-isothiazolinone, five-membered saturated heterocyclic ring structures containing a sulfur and a nitrogen in the 1-position and 2-positions respectively. Also known as: 4-amino-3-isothiazolidinone anabolism, 4-amino-3-isothiazolidinone biosynthesis, 4-amino-3-isothiazolidinone formation, 4-amino-3-isothiazolidinone synthesis Sources: GOC:jid